{
  "gene_name": "Contactin-6",
  "gene": "UniProtKB:Q9UQ52",
  "gene_symbol": "CNTN6",
  "term_label": "cell-cell adhesion mediator activity",
  "term_id": "GO:0098632"
}